negative regulation of type I hypersensitivity [GO:0001811] (biological process) Definition: Any process that stops, prevents, or reduces the rate of type I hypersensitivity, a type of inflammatory response. Sources: GOC:add, ISBN:0781735149 Also known as: down regulation of type I hypersensitivity, down-regulation of type I hypersensitivity, downregulation of type I hypersensitivity, inhibition of type I hypersensitivity Relationships: is a type of regulation of type I hypersensitivity [GO:0001810]; is a type of negative regulation of hypersensitivity [GO:0002884]; is a type of GO:0002890; negatively regulates type I hypersensitivity [GO:0016068]